protein localization to cell surface [GO:0034394] (biological process) Sources: GOC:mah Relationships: is a type of intracellular protein localization [GO:0008104] Regulation: regulated by regulation of protein localization to cell surface [GO:2000008]; negatively regulated by GO:2000009; positively regulated by positive regulation of protein localization to cell surface [GO:2000010] Definition: A process in which a protein is transported to, or maintained in, a location within the external part of the cell wall and/or plasma membrane. Also known as: protein localisation at cell surface, protein localization at cell surface